{
  "term_id": "GO:0016339",
  "term_label": "calcium-dependent cell-cell adhesion",
  "gene": "UniProtKB:P55291",
  "gene_name": "Cadherin-15",
  "gene_symbol": "CDH15"
}